{
  "term_label": "mitotic DNA replication initiation",
  "gene": "UniProtKB:P49736",
  "gene_symbol": "MCM2",
  "gene_name": "DNA replication licensing factor MCM2",
  "term_id": "GO:1902975"
}